{
  "gene_symbol": "MAGED1",
  "term_id": "GO:0005634",
  "term_label": "nucleus",
  "gene_name": "Melanoma-associated antigen D1",
  "gene": "UniProtKB:Q9Y5V3"
}